{
  "gene_symbol": "SLFN5",
  "gene": "UniProtKB:Q08AF3",
  "gene_name": "Schlafen family member 5",
  "term_label": "Unknown biological process",
  "term_id": "UNKNOWN:0002"
}